lycopene cleavage oxygenase activity [GO:0102818] (molecular function) Definition: Catalysis of the reaction: lycopene + 2 O2 = 2 sulcatone + bixin aldehyde. Sources: GOC:pz, MetaCyc:RXN-8236 Relationships: is a type of oxidoreductase activity, acting on single donors with incorporation of molecular oxygen, incorporation of one atom of oxygen (internal monooxygenases or internal mixed function oxidases) [GO:0016703]